negative regulation of hematopoietic stem cell proliferation [GO:1902034] (biological process) Definition: Any process that stops, prevents or reduces the frequency, rate or extent of hematopoietic stem cell proliferation. References: PMID:23403623 Sources: GOC:TermGenie Also known as: down regulation of hematopoietic stem cell proliferation, down regulation of hemopoietic stem cell proliferation, down-regulation of hematopoietic stem cell proliferation, down-regulation of hemopoietic stem cell proliferation, downregulation of hematopoietic stem cell proliferation, downregulation of hemopoietic stem cell proliferation, negative regulation of hemopoietic stem cell proliferation, inhibition of hematopoietic stem cell proliferation, inhibition of hemopoietic stem cell proliferation Relationships: is_a regulation of hematopoietic stem cell proliferation [GO:1902033]; is a type of negative regulation of hemopoiesis [GO:1903707]; is a type of negative regulation of stem cell proliferation [GO:2000647]; negatively regulates GO:0071425